calcitonin binding [GO:0032841] (molecular function) Sources: GOC:ecd Relationships: is a type of calcitonin family binding [GO:0097644] Definition: Binding to calcitonin, a peptide hormone responsible for reducing serum calcium levels by inhibiting osteoclastic bone reabsorption and promoting renal calcium excretion. It is synthesized and released by the C cells of the thyroid.